{
  "term_id": "GO:0007160",
  "gene": "UniProtKB:Q9UQP3",
  "term_label": "cell-matrix adhesion",
  "gene_name": "Tenascin-N",
  "gene_symbol": "TNN"
}